all-trans undecaprenol kinase activity [GO:0036432] (molecular function) Relationships: is a type of undecaprenol kinase activity [GO:0009038] Definition: Catalysis of the reaction: ATP + undecaprenol + all-trans-undecaprenyl phosphate + ADP + H+. Sources: RHEA:23752